{
  "term_id": "UNKNOWN:0001",
  "gene": "UniProtKB:Q8NBP0",
  "gene_symbol": "TTC13",
  "gene_name": "Tetratricopeptide repeat protein 13",
  "term_label": "Unknown molecular function"
}